{
  "gene_name": "Proteasome assembly chaperone 1",
  "term_id": "GO:0005783",
  "gene": "UniProtKB:O95456",
  "term_label": "endoplasmic reticulum",
  "gene_symbol": "PSMG1"
}